{
  "gene_name": "Nonsense-mediated mRNA decay factor SMG7",
  "gene": "UniProtKB:Q92540",
  "gene_symbol": "SMG7",
  "term_id": "GO:0070034",
  "term_label": "telomerase RNA binding"
}